negative regulation of penicillin catabolic process [GO:0033248] (BP) Also known as: negative regulation of penicillin breakdown, negative regulation of penicillin catabolism, negative regulation of penicillin degradation Sources: GOC:mah Definition: Any process that stops, prevents, or reduces the frequency, rate or extent of the chemical reactions and pathways leading to the breakdown of any antibiotic that contains the condensed beta-lactamthiazolidine ring system. Relationships: is a type of negative regulation of catabolic process [GO:0009895]; is a type of regulation of penicillin catabolic process [GO:0033247]; is a type of GO:0034249; is a type of negative regulation of small molecule metabolic process [GO:0062014]; negatively regulates penicillin catabolic process [GO:0042317]